{
  "gene": "UniProtKB:Q9H8X2",
  "term_id": "GO:0032958",
  "gene_name": "Inositol-pentakisphosphate 2-kinase",
  "term_label": "inositol phosphate biosynthetic process",
  "gene_symbol": "IPPK"
}